{
  "term_label": "Unknown biological process",
  "gene": "UniProtKB:Q8NH07",
  "term_id": "UNKNOWN:0002",
  "gene_symbol": "OR11H2",
  "gene_name": "Olfactory receptor 11H2"
}